{
  "gene": "UniProtKB:A0A1B0GVQ3",
  "gene_symbol": "CCDC200",
  "term_label": "Unknown biological process",
  "term_id": "UNKNOWN:0002",
  "gene_name": "Coiled-coil domain-containing protein 200"
}